positive regulation of dehydroaustinol biosynthetic process [GO:1900651] (biological process) Relationships: is a type of positive regulation of secondary metabolite biosynthetic process [GO:1900378]; is a type of regulation of dehydroaustinol biosynthetic process [GO:1900649]; positively regulates GO:1900563 Sources: GOC:TermGenie, GOC:di Also known as: activation of dehydroaustinol anabolism, activation of dehydroaustinol biosynthesis, activation of dehydroaustinol formation, activation of dehydroaustinol synthesis, positive regulation of dehydroaustinol anabolism, positive regulation of dehydroaustinol biosynthesis, positive regulation of dehydroaustinol formation, positive regulation of dehydroaustinol synthesis, up regulation of dehydroaustinol anabolism, up regulation of dehydroaustinol biosynthesis, up regulation of dehydroaustinol biosynthetic process, up regulation of dehydroaustinol formation, up regulation of dehydroaustinol synthesis, up-regulation of dehydroaustinol anabolism, up-regulation of dehydroaustinol biosynthesis, up-regulation of dehydroaustinol biosynthetic process, up-regulation of dehydroaustinol formation, up-regulation of dehydroaustinol synthesis, upregulation of dehydroaustinol anabolism, upregulation of dehydroaustinol biosynthesis, upregulation of dehydroaustinol biosynthetic process, upregulation of dehydroaustinol formation, upregulation of dehydroaustinol synthesis, activation of dehydroaustinol biosynthetic process Definition: Any process that activates or increases the frequency, rate or extent of dehydroaustinol biosynthetic process.